{
  "term_label": "kinesin complex",
  "gene_symbol": "KIF3C",
  "term_id": "GO:0005871",
  "gene_name": "Kinesin-like protein KIF3C",
  "gene": "UniProtKB:O14782"
}